{
  "gene_symbol": "LINC02898",
  "term_id": "UNKNOWN:0002",
  "term_label": "Unknown biological process",
  "gene": "UniProtKB:Q6ZV80",
  "gene_name": "Putative uncharacterized protein LINC02898"
}